{
  "term_id": "UNKNOWN:0001",
  "gene_symbol": "NPIPB9",
  "term_label": "Unknown molecular function",
  "gene_name": "Nuclear pore complex-interacting protein family member B9",
  "gene": "UniProtKB:F8W1W9"
}